{
  "gene_name": "Myb-related transcription factor, partner of profilin",
  "term_id": "GO:0000981",
  "term_label": "DNA-binding transcription factor activity, RNA polymerase II-specific",
  "gene_symbol": "MYPOP",
  "gene": "UniProtKB:Q86VE0"
}